{
  "gene_symbol": "STX1B",
  "gene_name": "Syntaxin-1B",
  "term_label": "SNAP receptor activity",
  "gene": "UniProtKB:P61266",
  "term_id": "GO:0005484"
}